mitotic telomere tethering at nuclear periphery [GO:0044820] (BP) References: PMID:25778919 Sources: GOC:mtg_cell_cycle Definition: The process in which a telomere is maintained in a specific location at the nuclear periphery, as part of a mitotic cell cycle. Relationships: is a type of telomere tethering at nuclear periphery [GO:0034398]; is part of mitotic telomere clustering and tethering at nuclear periphery [GO:0120109] Regulation: regulated by regulation of mitotic telomere tethering at nuclear periphery [GO:1904536]; negatively regulated by negative regulation of mitotic telomere tethering at nuclear periphery [GO:1904537]